regulation of oocyte maturation [GO:1900193] (biological process) Relationships: is a type of GO:1903429; is a type of GO:2000241; regulates oocyte maturation [GO:0001556] Subtypes: GO:1900194, GO:1900195 Definition: Any process that modulates the frequency, rate or extent of oocyte maturation. Sources: GOC:TermGenie, GOC:kmv